{
  "gene_name": "HIG1 domain family member 1C",
  "gene": "UniProtKB:A8MV81",
  "term_label": "Unknown molecular function",
  "term_id": "UNKNOWN:0001",
  "gene_symbol": "HIGD1C"
}